chitobiosyldiphosphodolichol beta-mannosyltransferase activity [GO:0004578] (MF) Definition: Catalysis of the reaction: an N,N'-diacetylchitobiosyl-diphospho-di-trans,poly-cis-dolichol + GDP-alpha-D-mannose = a beta-D-Man-(1->4)-beta-D-GlcNAc-(1->4)-alpha-D-GlcNAc-diphospho-di-trans,poly-cis-dolichol + GDP + H+. Sources: RHEA:13865 Also known as: GDP-mannose-dolichol diphosphochitobiose mannosyltransferase activity, GDP-mannose:chitobiosyldiphosphodolichol beta-D-mannosyltransferase activity, guanosine diphosphomannose-dolichol diphosphochitobiose mannosyltransferase activity Relationships: is a type of beta-1,4-mannosyltransferase activity [GO:0019187]; is a type of GlcNAc(2)-PP-Dol mannosyltransferase activity [GO:0120562]